{
  "term_id": "GO:0005525",
  "term_label": "GTP binding",
  "gene_symbol": "RAB39A",
  "gene_name": "Ras-related protein Rab-39A",
  "gene": "UniProtKB:Q14964"
}